{
  "gene": "UniProtKB:Q68D85",
  "term_id": "UNKNOWN:0003",
  "gene_name": "Natural cytotoxicity triggering receptor 3 ligand 1",
  "gene_symbol": "NCR3LG1",
  "term_label": "Unknown cellular component"
}